{
  "term_id": "UNKNOWN:0002",
  "gene_name": "Translocator protein",
  "gene": "UniProtKB:P30536",
  "term_label": "Unknown biological process",
  "gene_symbol": "TSPO"
}